{
  "gene": "UniProtKB:O00299",
  "term_id": "GO:0005737",
  "term_label": "cytoplasm",
  "gene_symbol": "CLIC1",
  "gene_name": "Chloride intracellular channel protein 1"
}